lipopolysaccharide core heptosyltransferase activity [GO:0071967] (molecular function) Sources: MetaCyc:RXN0-5122 Relationships: is a type of lipopolysaccharide heptosyltransferase activity [GO:0008920] Also known as: LPS core heptosyltransferase activity Definition: Catalysis of the reaction: glucosyl-heptosyl2-KDO2-lipid A-phosphate + ADP-L-glycero-beta-D-manno-heptose = glucosyl-heptosyl3-KDO2-lipid A-phosphate + ADP + H+.